{
  "term_label": "cilium assembly",
  "term_id": "GO:0060271",
  "gene_symbol": "RILPL2",
  "gene_name": "RILP-like protein 2",
  "gene": "UniProtKB:Q969X0"
}